{
  "gene_symbol": "ASPH",
  "gene": "UniProtKB:Q12797",
  "term_label": "regulation of cytosolic calcium ion concentration",
  "term_id": "GO:0051480",
  "gene_name": "Aspartyl_asparaginyl beta-hydroxylase"
}